junctional membrane complex [GO:0030314] (cellular component) Relationships: is a type of protein-containing complex [GO:0032991]; is part of sarcoplasm [GO:0016528] Definition: Complex formed in muscle cells between the membrane of the sarcoplasmic reticulum and invaginations of the plasma membrane (T-tubules). Also known as: triad junction References: PMID:11535622